{
  "gene": "UniProtKB:Q8WV16",
  "term_id": "GO:0080008",
  "term_label": "Cul4-RING E3 ubiquitin ligase complex",
  "gene_name": "DDB1- and CUL4-associated factor 4",
  "gene_symbol": "DCAF4"
}